antigen processing and presentation following receptor mediated endocytosis [GO:0002751] (biological process) Subtypes: B cell antigen processing and presentation mediated by B cell receptor uptake of antigen [GO:0002417] Sources: GOC:add, ISBN:0781735149 Definition: Antigen processing and presentation which is initiated by uptake of antigen receptor-mediated endocytosis. Relationships: is a type of GO:0002745